G protein-coupled enkephalin receptor activity [GO:0038046] (molecular function) Relationships: is a type of G protein-coupled opioid receptor activity [GO:0004985]; is a type of G protein-coupled peptide receptor activity [GO:0008528] Sources: GOC:bf, Wikipedia:Enkephalin Also known as: enkephalin receptor activity, delta-opioid receptor activity Definition: Combining with an enkephalin, and transmitting the signal across the membrane by activating an associated G-protein. A enkephalin is a pentapeptide (Tyr-Gly-Gly-Phe-Met or Tyr-Gly-Gly-Phe-Leu) involved in regulating nociception in the body.